{
  "gene_symbol": "KBTBD6",
  "gene_name": "Kelch repeat and BTB domain-containing protein 6",
  "term_label": "Cul3-RING ubiquitin ligase complex",
  "term_id": "GO:0031463",
  "gene": "UniProtKB:Q86V97"
}